{
  "gene": "UniProtKB:Q52WX2",
  "term_label": "Unknown cellular component",
  "gene_symbol": "SBK1",
  "gene_name": "Serine_threonine-protein kinase SBK1",
  "term_id": "UNKNOWN:0003"
}